{
  "term_label": "positive regulation of RIG-I signaling pathway",
  "gene_name": "Zinc finger CCCH-type antiviral protein 1",
  "gene_symbol": "ZC3HAV1",
  "gene": "UniProtKB:Q7Z2W4",
  "term_id": "GO:1900246"
}